L-malate dehydrogenase (quinone) activity [GO:0008924] (molecular function) References: PMID:234747 Sources: RHEA:46012 Relationships: is a type of malate dehydrogenase activity [GO:0016615]; is a type of oxidoreductase activity, acting on the CH-OH group of donors, quinone or similar compound as acceptor [GO:0016901] Also known as: MQO activity, (S)-malate:(quinone) oxidoreductase activity, (S)-malate:quinone oxidoreductase activity, FAD-dependent malate dehydrogenase activity Definition: Catalysis of the reaction: (S)-malate + a quinone = oxaloacetate + a quinol. Vitamin K (menaquinone) and several other quinones can act as acceptors.